{
  "gene_name": "Alpha-2-macroglobulin-like protein 1",
  "term_id": "UNKNOWN:0002",
  "term_label": "Unknown biological process",
  "gene_symbol": "A2ML1",
  "gene": "UniProtKB:A8K2U0"
}